{
  "gene_name": "Interferon-induced transmembrane protein 10",
  "gene": "UniProtKB:A6NMD0",
  "term_label": "plasma membrane",
  "gene_symbol": "IFITM10",
  "term_id": "GO:0005886"
}